{
  "gene_symbol": "KIR2DS5",
  "term_id": "GO:0004888",
  "gene": "UniProtKB:Q14953",
  "gene_name": "Killer cell immunoglobulin-like receptor 2DS5",
  "term_label": "transmembrane signaling receptor activity"
}